{
  "term_id": "GO:0005737",
  "gene_symbol": "OPHN1",
  "gene": "UniProtKB:O60890",
  "term_label": "cytoplasm",
  "gene_name": "Oligophrenin-1"
}